{
  "term_id": "UNKNOWN:0003",
  "gene": "UniProtKB:A0A1B0GU71",
  "gene_name": "Uncharacterized protein CFAP97D2",
  "gene_symbol": "CFAP97D2",
  "term_label": "Unknown cellular component"
}